(3S)-(+)-asterisca-2(9),6-diene synthase activity [GO:0120086] (molecular function) References: PMID:27862766 Also known as: asterisca-2(9),6-diene synthase activity Relationships: is a type of sesquiterpene synthase activity [GO:0010334] Definition: Catalysis of the reaction: 2-trans,6-trans-farnesyl diphosphate = diphosphate + (3S)-(+)-asterisca-2(9),6-diene.